mast cell homeostasis [GO:0033023] (biological process) Note: Note that this term represents the return of mast cell levels to stable numbers following an immune response as well as the proliferation and elimination of mast cells required to maintain stable numbers in the absence of an outside stimulus. References: PMID:11292031 Sources: GOC:add Definition: The process of regulating the proliferation and elimination of mast cells such that the total number of mast cells within a whole or part of an organism is stable over time in the absence of an outside stimulus. Relationships: is a type of GO:0001776; is a type of myeloid cell homeostasis [GO:0002262]